{
  "gene_symbol": "CLDN23",
  "gene": "UniProtKB:Q96B33",
  "term_id": "UNKNOWN:0002",
  "gene_name": "Claudin-23",
  "term_label": "Unknown biological process"
}